phosphatidylinositol dephosphorylation [GO:0046856] (biological process) Regulation: regulated by regulation of phosphatidylinositol dephosphorylation [GO:0060304] Relationships: is a type of phosphatidylinositol metabolic process [GO:0046488]; is a type of phospholipid dephosphorylation [GO:0046839] Definition: The process of removing one or more phosphate groups from a phosphatidylinositol. Sources: ISBN:0198506732 Also known as: phosphoinositide dephosphorylation, PIP catabolism, PtdInsP catabolism, PtdInsP dephosphorylation, phosphatidylinositol phosphate catabolic process, phosphatidylinositol phosphate dephosphorylation